{
  "gene": "UniProtKB:P03897",
  "gene_name": "NADH-ubiquinone oxidoreductase chain 3",
  "gene_symbol": "MT-ND3",
  "term_id": "UNKNOWN:0002",
  "term_label": "Unknown biological process"
}